{
  "term_label": "glycolipid translocation",
  "gene_symbol": "RFT1",
  "gene_name": "Protein RFT1 homolog",
  "term_id": "GO:0034203",
  "gene": "UniProtKB:Q96AA3"
}